venom-mediated perturbation of signal transduction [GO:0044509] (biological process) Also known as: envenomation resulting in modulation of signal transduction in another organism, envenomation resulting in modulation of signal transduction in other organismm Subtypes: venom-mediated perturbation of G protein-coupled receptor signaling pathway [GO:0044513], venom-mediated vasodilation by activation of nitric oxide-cGMP-mediated signaling [GO:0140165], GO:0140166 References: PMID:8405712 Sources: GOC:fj, GOC:jl Definition: A process in which an organism alters or subverts a signal transduction pathway in another organism via the action of a venom. Relationships: is a type of GO:0035738